protein import into peroxisome membrane [GO:0045046] (biological process) References: PMID:11687502 Sources: ISBN:0716731363 Also known as: peroxisome membrane protein import, protein transport into peroxisome membrane Relationships: is a type of GO:0006886; is a type of peroxisomal membrane transport [GO:0015919]; is a type of GO:0072657; is a type of protein localization to peroxisome [GO:0072662]; is a type of GO:0072663; is a type of establishment of protein localization to membrane [GO:0090150] Definition: The targeting of proteins into the peroxisomal membrane. The process is not well understood, but both signals and mechanism differ from those involved in peroxisomal matrix protein import.